syringetin 3-O-methyltransferase activity [GO:0102442] (molecular function) Relationships: is a type of GO:0008168 Sources: RHEA:74767 Definition: Catalysis of the reaction: S-adenosyl-L-methionine + syringetin = 3,3',5'-O-trimethylmyricetin + H(+) + S-adenosyl-L-homocysteine.